gap junction channel activity involved in Purkinje myocyte-ventricular cardiac muscle cell electrical coupling [GO:0086079] (MF) Definition: A wide pore channel activity that enables a direct cytoplasmic connection from a Purkinje myocyte to a ventricular cardiac muscle cell. The gap junction passes electrical signals between the cells contributing to cardiac conduction. Sources: GOC:BHF, GOC:mtg_cardiac_conduct_nov11 Relationships: is a type of gap junction channel activity involved in cardiac conduction electrical coupling [GO:0086075]; is part of Purkinje myocyte to ventricular cardiac muscle cell communication by electrical coupling [GO:0086055]